regulation of male germ-line stem cell asymmetric division [GO:1904838] (biological process) Relationships: is a type of regulation of asymmetric cell division [GO:0009786]; is a type of GO:0051239; is a type of regulation of stem cell division [GO:2000035]; regulates male germ-line stem cell asymmetric division [GO:0048133] Definition: Any process that modulates the frequency, rate or extent of male germ-line stem cell asymmetric division. Subtypes: GO:1904839, GO:1904840 References: PMID:19339709 Sources: GOC:TermGenie, GO_REF:0000058 Also known as: regulation of male germ-line stem cell renewal